{
  "gene_symbol": "GAS2",
  "gene": "UniProtKB:O43903",
  "term_id": "GO:0051015",
  "term_label": "actin filament binding",
  "gene_name": "Growth arrest-specific protein 2"
}